{
  "gene_name": "AP-2 complex subunit alpha-2",
  "term_label": "AP-2 adaptor complex",
  "term_id": "GO:0030122",
  "gene_symbol": "AP2A2",
  "gene": "UniProtKB:O94973"
}